{
  "gene_symbol": "Q96IR3",
  "gene_name": "Putative uncharacterized protein MGC15705",
  "term_label": "Unknown biological process",
  "gene": "UniProtKB:Q96IR3",
  "term_id": "UNKNOWN:0002"
}